{
  "term_label": "regulation of transcription by RNA polymerase II",
  "term_id": "GO:0006357",
  "gene_symbol": "ELK1",
  "gene": "UniProtKB:P19419",
  "gene_name": "ETS domain-containing protein Elk-1"
}